{
  "gene": "UniProtKB:Q659A1",
  "term_label": "Unknown molecular function",
  "gene_symbol": "ICE2",
  "term_id": "UNKNOWN:0001",
  "gene_name": "Little elongation complex subunit 2"
}